{
  "gene_name": "Receptor-type tyrosine-protein phosphatase S",
  "term_label": "protein tyrosine phosphatase activity",
  "gene": "UniProtKB:Q13332",
  "gene_symbol": "PTPRS",
  "term_id": "GO:0004725"
}